{
  "term_id": "GO:0005737",
  "term_label": "cytoplasm",
  "gene": "UniProtKB:P35520",
  "gene_symbol": "CBS",
  "gene_name": "Cystathionine beta-synthase"
}